{
  "term_id": "GO:0051604",
  "gene_name": "Kallikrein-6",
  "gene_symbol": "KLK6",
  "term_label": "protein maturation",
  "gene": "UniProtKB:Q92876"
}